detoxification of cobalt ion [GO:0010299] (biological process) Definition: Any process that reduces or removes the toxicity of cobalt ion (Co2+). These include transport of cobalt away from sensitive areas and to compartments or complexes whose purpose is sequestration of cobalt ion. Relationships: is a type of detoxification of inorganic compound [GO:0061687]; is part of response to cobalt ion [GO:0032025] Sources: GOC:tair_curators